negative regulation of plant-type hypersensitive response [GO:0034051] (biological process) Sources: GOC:pamgo_curators Relationships: is a type of regulation of plant-type hypersensitive response [GO:0010363]; is a type of GO:0043069; is a type of GO:0045824; negatively regulates plant-type hypersensitive response [GO:0009626] Definition: Any process that stops, prevents, or reduces the frequency, rate or extent of the hypersensitive response in a plant. Also known as: down regulation of plant-type hypersensitive response, down-regulation of plant-type hypersensitive response, downregulation of plant-type hypersensitive response, negative regulation of HR, negative regulation of HR-PCD, negative regulation of plant hypersensitive response, inhibition of plant-type hypersensitive response